{
  "gene_name": "N-alpha-acetyltransferase 30",
  "term_id": "GO:0004596",
  "term_label": "protein-N-terminal amino-acid acetyltransferase activity",
  "gene": "UniProtKB:Q147X3",
  "gene_symbol": "NAA30"
}